prenyltransferase activity [GO:0004659] (MF) Sources: GOC:mah Subtypes: GO:0008318, 4-hydroxybenzoate polyprenyltransferase activity [GO:0008412], GO:0008495, GO:0010354, chlorophyll synthetase activity [GO:0046408], 1,4-dihydroxy-2-naphthoate polyprenyltransferase activity [GO:0046428], 15-cis-phytoene synthase activity [GO:0046905], GO:0047294, geranylgeranylglycerol-phosphate geranylgeranyltransferase activity [GO:0047295], squalene synthase [NAD(P)H] activity [GO:0051996], flavin prenyltransferase activity [GO:0106141], prenyl diphosphate synthase activity [GO:0120531], heptaprenylglyceryl phosphate synthase activity [GO:0120536], menadiol geranylgeranyltransferase activity [GO:0120566] Relationships: is a type of transferase activity, transferring alkyl or aryl (other than methyl) groups [GO:0016765] Definition: Catalysis of the transfer of a prenyl group from one compound (donor) to another (acceptor).